{
  "term_label": "RNA polymerase II transcription regulatory region sequence-specific DNA binding",
  "gene_name": "Zinc finger protein 433",
  "gene_symbol": "ZNF433",
  "term_id": "GO:0000977",
  "gene": "UniProtKB:Q8N7K0"
}